{
  "gene_symbol": "ZNF320",
  "gene_name": "Zinc finger protein 320",
  "gene": "UniProtKB:A2RRD8",
  "term_id": "GO:0006357",
  "term_label": "regulation of transcription by RNA polymerase II"
}